NADH dehydrogenase (menaquinone) (non-electrogenic) activity [GO:0103036] (molecular function) Relationships: is a type of NADH dehydrogenase (quinone) (non-electrogenic) activity [GO:0050136] Definition: Catalysis of the reaction: a menaquinone + NADH + H+ = a menaquinol + NAD+. Also known as: NADH:menaquinone oxidoreductase activity Sources: RHEA:29235